host cell late endosome [GO:0044184] (cellular component) Sources: GOC:jl Definition: A prelysosomal endocytic organelle differentiated from host early endosomes by lower lumenal pH and different protein composition. Host late endosomes are more spherical than early endosomes and are mostly juxtanuclear, being concentrated near the microtubule organizing center. Subtypes: host multivesicular body [GO:0072494] Relationships: is a type of host cell endosome [GO:0044174]